{
  "gene_symbol": "STEAP4",
  "term_label": "cupric reductase (NADH) activity",
  "term_id": "GO:0008823",
  "gene": "UniProtKB:Q687X5",
  "gene_name": "Metalloreductase STEAP4"
}